beak morphogenesis [GO:0071729] (biological process) Relationships: is a type of anatomical structure morphogenesis [GO:0009653]; is part of beak development [GO:0071728] Definition: The process in which the anatomical structures of the beak are generated and organized. The avian beak is an external anatomical structure, in the head region, that is adapted for feeding self and young, catching prey, probing, etc. It encompasses, but is not restricted to, the maxilla, mandible, maxillary rhamphotheca, mandibular rhamphotheca, nostril, nasal fossa, nasal bones, egg tooth and rictus. Sources: GOC:lp, ISBN:0702008729